{
  "gene": "UniProtKB:Q5VST6",
  "gene_name": "Alpha_beta hydrolase domain-containing protein 17B",
  "term_id": "GO:1905668",
  "term_label": "positive regulation of protein localization to endosome",
  "gene_symbol": "ABHD17B"
}